regulation of synaptic vesicle docking [GO:0099148] (biological process) Sources: GOC:dos Relationships: is_a regulation of vesicle docking [GO:0106020]; regulates synaptic vesicle docking [GO:0016081] Definition: Any process that modulates the frequency, rate or extent of synaptic vesicle docking.